{
  "term_id": "GO:0045039",
  "term_label": "protein insertion into mitochondrial inner membrane",
  "gene": "UniProtKB:P62072",
  "gene_name": "Mitochondrial import inner membrane translocase subunit Tim10",
  "gene_symbol": "TIMM10"
}